{
  "gene_name": "Dachshund homolog 1",
  "term_label": "regulation of transcription by RNA polymerase II",
  "gene": "UniProtKB:Q9UI36",
  "term_id": "GO:0006357",
  "gene_symbol": "DACH1"
}